BMP secretion [GO:0038055] (biological process) Sources: GOC:sart Also known as: BMP protein secretion, bone morphogenetic protein secretion Definition: The controlled release of a member of the BMP family of proteins from a cell. Regulation: positively regulated by positive regulation of BMP secretion [GO:1900144]; regulated by regulation of BMP secretion [GO:2001284]; negatively regulated by negative regulation of BMP secretion [GO:2001285] Relationships: is a type of protein secretion [GO:0009306]; is a type of signal release [GO:0023061]